notochord cell differentiation [GO:0060034] (biological process) Sources: GOC:dph Relationships: is a type of GO:0030154; is part of notochord development [GO:0030903] Definition: The process in which relatively unspecialized cells acquire specialized structural and/or functional features cells that make up the notochord. Differentiation includes the processes involved in commitment of a cell to a notochord cell fate.